{
  "gene_name": "RNA-binding protein 41",
  "term_label": "pre-mRNA intronic binding",
  "term_id": "GO:0097157",
  "gene_symbol": "RBM41",
  "gene": "UniProtKB:Q96IZ5"
}